{
  "gene": "UniProtKB:Q6DJT9",
  "term_label": "Unknown cellular component",
  "term_id": "UNKNOWN:0003",
  "gene_symbol": "PLAG1",
  "gene_name": "Zinc finger protein PLAG1"
}